cerebellar granular layer morphogenesis [GO:0021683] (biological process) Definition: The process in which the anatomical structure of the cerebellar granular layer is generated and organized. The granular layer is the innermost layer of the cerebellar cortex. This layer contains densely packed small neurons, mostly granule cells. Some Golgi cells are found at the outer border. Granule neurons send parallel fibers to the upper molecular layer, where they synapse with Purkinje cell dendrites. Mossy fibers from the pontine nuclei in the white matter synapse with granule cell axons, Golgi cell axons and unipolar brush interneuron axons at cerebellar glomeruli in the granule cell layer. Relationships: is a type of anatomical structure morphogenesis [GO:0009653]; BFO_0000050 cerebellar granular layer development [GO:0021681]; is part of cerebellar cortex morphogenesis [GO:0021696] Sources: GOC:cls, GOC:dgh, GOC:dph, GOC:jid, GO_REF:0000021